{
  "gene": "UniProtKB:P98172",
  "term_label": "ephrin receptor signaling pathway",
  "gene_name": "Ephrin-B1",
  "gene_symbol": "EFNB1",
  "term_id": "GO:0048013"
}